oxidoreductase activity, acting on single donors with incorporation of molecular oxygen [GO:0016701] (molecular function) Sources: EC:1.13.-.- Definition: Catalysis of an oxidation-reduction (redox) reaction in which hydrogen or electrons are transferred from one donor, and molecular oxygen is incorporated into a donor. Also known as: oxygenase, oxidoreductase activity, acting on single donors with incorporation of molecular oxygen, miscellaneous Relationships: is a type of GO:0016491 Subtypes: oxidoreductase activity, acting on single donors with incorporation of molecular oxygen, incorporation of two atoms of oxygen [GO:0016702], oxidoreductase activity, acting on single donors with incorporation of molecular oxygen, incorporation of one atom of oxygen (internal monooxygenases or internal mixed function oxidases) [GO:0016703], 1,2-dihydroxynaphthalene dioxygenase activity [GO:0018554], inositol oxygenase activity [GO:0050113], tryptophan 2'-dioxygenase activity [GO:0050360]